{
  "gene_name": "ZW10 interactor",
  "gene_symbol": "ZWINT",
  "gene": "UniProtKB:O95229",
  "term_label": "dendrite",
  "term_id": "GO:0030425"
}